{
  "gene_symbol": "EIF2B3",
  "term_id": "GO:0005851",
  "term_label": "eukaryotic translation initiation factor 2B complex",
  "gene": "UniProtKB:Q9NR50",
  "gene_name": "Translation initiation factor eIF-2B subunit gamma"
}